regulation of substrate-dependent cell migration, cell attachment to substrate [GO:1904235] (biological process) Relationships: is a type of regulation of cell-substrate adhesion [GO:0010810]; is a type of regulation of cell migration [GO:0030334]; regulates substrate-dependent cell migration, cell attachment to substrate [GO:0006931] Definition: Any process that modulates the frequency, rate or extent of substrate-dependent cell migration, cell attachment to substrate. Subtypes: negative regulation of substrate-dependent cell migration, cell attachment to substrate [GO:1904236], GO:1904237 Also known as: regulation of substrate-bound cell migration, cell attachment to substrate References: PMID:25834989 Sources: GOC:TermGenie, GO_REF:0000058